{
  "term_id": "UNKNOWN:0003",
  "gene_symbol": "TAB2",
  "term_label": "Unknown cellular component",
  "gene": "UniProtKB:Q9NYJ8",
  "gene_name": "TGF-beta-activated kinase 1 and MAP3K7-binding protein 2"
}